{
  "term_id": "UNKNOWN:0003",
  "term_label": "Unknown cellular component",
  "gene_name": "Transcriptional repressor RHIT",
  "gene": "UniProtKB:O95201",
  "gene_symbol": "ZNF205"
}